{
  "gene_symbol": "RNASE6",
  "term_id": "GO:0050830",
  "gene_name": "Ribonuclease K6",
  "term_label": "defense response to Gram-positive bacterium",
  "gene": "UniProtKB:Q93091"
}